{
  "term_label": "negative regulation of transcription by RNA polymerase II",
  "gene": "UniProtKB:P14373",
  "gene_name": "Zinc finger protein RFP",
  "term_id": "GO:0000122",
  "gene_symbol": "TRIM27"
}